astral microtubule anchoring at mitotic spindle pole body [GO:1990734] (biological process) Definition: Any process in which an astral microtubule is maintained in a specific location in a cell by attachment to a mitotic spindle pole body. Microtubules attach to spindle pole bodies at the minus end. Relationships: is a type of microtubule anchoring at spindle pole body [GO:0034631] References: PMID:15004232